farnesyl diphosphate catabolic process [GO:0045339] (biological process) Relationships: is a type of phospholipid catabolic process [GO:0009395]; is a type of terpenoid catabolic process [GO:0016115]; is a type of farnesyl diphosphate metabolic process [GO:0045338] Sources: GOC:go_curators Also known as: farnesyl diphosphate breakdown, farnesyl diphosphate catabolism, farnesyl diphosphate degradation Definition: The chemical reactions and pathways resulting in the breakdown of farnesyl diphosphate.